positive regulation of compound eye photoreceptor development [GO:0045315] (biological process) Definition: Any process that activates or increases the frequency, rate or extent of compound eye photoreceptor development. Relationships: is a type of positive regulation of eye photoreceptor cell development [GO:0042479]; is a type of GO:0045314; positively regulates GO:0042051 Also known as: activation of eye photoreceptor development, positive regulation of eye photoreceptor development, stimulation of eye photoreceptor development, up regulation of eye photoreceptor development, up-regulation of eye photoreceptor development, upregulation of eye photoreceptor development Sources: GOC:bf